{
  "gene_name": "Receptor expression-enhancing protein 6",
  "gene": "UniProtKB:Q96HR9",
  "term_label": "Unknown cellular component",
  "gene_symbol": "REEP6",
  "term_id": "UNKNOWN:0003"
}